{
  "gene": "UniProtKB:P15153",
  "term_id": "GO:0042995",
  "term_label": "cell projection",
  "gene_symbol": "RAC2",
  "gene_name": "Ras-related C3 botulinum toxin substrate 2"
}